semaphorin-plexin signaling pathway [GO:0071526] (biological process) Relationships: is a type of cell surface receptor signaling pathway [GO:0007166] Regulation: regulated by regulation of semaphorin-plexin signaling pathway [GO:2001260]; RO_0002212 by negative regulation of semaphorin-plexin signaling pathway [GO:2001261]; positively regulated by positive regulation of semaphorin-plexin signaling pathway [GO:2001262] References: PMID:15239959 Sources: GOC:BHF, GOC:mah, GOC:vk Definition: The series of molecular signals generated as a consequence of a semaphorin receptor (composed of a plexin and a neurophilin) binding to a semaphorin ligand. Subtypes: semaphorin-plexin signaling pathway involved in outflow tract morphogenesis [GO:0071527], GO:1900220, semaphorin-plexin signaling pathway involved in neuron projection guidance [GO:1902285], semaphorin-plexin signaling pathway involved in regulation of photoreceptor cell axon guidance [GO:2000305] Also known as: semaphorin-plexin signalling pathway